{
  "gene_symbol": "LYPD1",
  "gene": "UniProtKB:Q8N2G4",
  "term_id": "GO:0030550",
  "gene_name": "Ly6_PLAUR domain-containing protein 1",
  "term_label": "acetylcholine receptor inhibitor activity"
}